negative regulation of methane biosynthetic process from methylamine [GO:1900349] (biological process) Also known as: down regulation of methane biosynthetic process from methylamine, down-regulation of methane biosynthetic process from methylamine, downregulation of methane biosynthetic process from methylamine, inhibition of methane biosynthetic process from methylamine Relationships: is a type of negative regulation of amine metabolic process [GO:0033239]; is a type of regulation of methane biosynthetic process from methylamine [GO:1900348]; is a type of negative regulation of alkane biosynthetic process [GO:1901578]; is a type of GO:1901856; negatively regulates GO:2001128 Definition: Any process that stops, prevents or reduces the frequency, rate or extent of methane biosynthetic process from methylamine. Sources: GOC:TermGenie, GOC:mengo_curators